negative regulation of glucuronoxylan catabolic process [GO:2000916] (biological process) Also known as: negative regulation of glucuronoxylan catabolism Subtypes: negative regulation of glucuronoarabinoxylan catabolic process [GO:2000919] Definition: Any process that stops, prevents or reduces the frequency, rate or extent of glucuronoxylan catabolic process. Sources: GOC:mengo_curators Relationships: is a type of regulation of glucuronoxylan catabolic process [GO:2000915]; is a type of negative regulation of xylan catabolic process [GO:2001001]; negatively regulates glucuronoxylan catabolic process [GO:2000886]